{
  "gene": "UniProtKB:O15111",
  "gene_name": "Inhibitor of nuclear factor kappa-B kinase subunit alpha",
  "term_label": "positive regulation of transcription by RNA polymerase II",
  "gene_symbol": "CHUK",
  "term_id": "GO:0045944"
}